{
  "gene": "UniProtKB:Q9NZQ7",
  "gene_symbol": "CD274",
  "term_label": "immune response",
  "term_id": "GO:0006955",
  "gene_name": "Programmed cell death 1 ligand 1"
}